{
  "term_label": "positive regulation of exocytosis",
  "gene_name": "Exophilin-5",
  "gene_symbol": "EXPH5",
  "term_id": "GO:0045921",
  "gene": "UniProtKB:Q8NEV8"
}